{
  "term_label": "regulation of mitochondrial fission",
  "term_id": "GO:0090140",
  "gene_name": "E3 ubiquitin-protein ligase MARCHF5",
  "gene_symbol": "MARCHF5",
  "gene": "UniProtKB:Q9NX47"
}